{
  "term_label": "nucleus",
  "term_id": "GO:0005634",
  "gene": "UniProtKB:Q8IZA3",
  "gene_symbol": "H1-8",
  "gene_name": "Histone H1.8"
}